{
  "gene": "UniProtKB:Q9Y692",
  "gene_symbol": "GMEB1",
  "term_label": "nucleus",
  "gene_name": "Glucocorticoid modulatory element-binding protein 1",
  "term_id": "GO:0005634"
}